pyridoxamine-pyruvate transaminase activity [GO:0047300] (molecular function) Sources: EC:2.6.1.30, RHEA:12841 Definition: Catalysis of the reaction: pyridoxamine + pyruvate = L-alanine + pyridoxal. Also known as: pyridoxamine-pyruvic transaminase, pyridoxamine-pyruvate aminotransferase activity, pyridoxamine--pyruvate aminotransferase activity, pyridoxamine:pyruvate aminotransferase activity, pyridoxamineu-pyruvic transaminase activity Relationships: is a type of transaminase activity [GO:0008483]